{
  "gene": "UniProtKB:Q86WJ1",
  "term_label": "chromatin remodeling",
  "term_id": "GO:0006338",
  "gene_symbol": "CHD1L",
  "gene_name": "Chromodomain-helicase-DNA-binding protein 1-like"
}